glutamate biosynthetic process [GO:0006537] (biological process) Relationships: is a type of GO:0006536; is a type of glutamine family amino acid biosynthetic process [GO:0009084]; is a type of GO:0043650 Also known as: glutamate anabolism, glutamate biosynthesis, glutamate formation, glutamate synthesis, glutamic acid biosynthesis, glutamic acid biosynthetic process, glutamate biosynthesis, using glutamate dehydrogenase (NAD(P)+), glutamate biosynthesis, using glutamate synthase (NADPH), glutamate biosynthetic process, using glutamate dehydrogenase (NAD(P)+), glutamate biosynthetic process, using glutamate synthase (NADPH) Definition: The chemical reactions and pathways resulting in the formation of glutamate, the anion of 2-aminopentanedioic acid. Subtypes: L-glutamate biosynthetic process [GO:0097054] Sources: GOC:go_curators